cAMP metabolic process [GO:0046058] (biological process) Definition: The chemical reactions and pathways involving the nucleotide cAMP (cyclic AMP, adenosine 3',5'-cyclophosphate). Also known as: 3',5' cAMP metabolic process, 3',5' cAMP metabolism, 3',5'-cAMP metabolic process, 3',5'-cAMP metabolism, adenosine 3',5'-cyclophosphate metabolic process, adenosine 3',5'-cyclophosphate metabolism, cAMP metabolism, cyclic AMP metabolic process, cyclic AMP metabolism, cAMP generating peptide activity Relationships: is a type of purine ribonucleotide metabolic process [GO:0009150]; is a type of cyclic purine nucleotide metabolic process [GO:0052652] Sources: GOC:go_curators Subtypes: cAMP biosynthetic process [GO:0006171], cAMP catabolic process [GO:0006198]